{
  "term_id": "GO:0016020",
  "gene_name": "Drebrin-like protein",
  "gene": "UniProtKB:Q9UJU6",
  "gene_symbol": "DBNL",
  "term_label": "membrane"
}